{
  "gene_name": "Sperm acrosome membrane-associated protein 3",
  "term_label": "sperm flagellum",
  "gene_symbol": "SPACA3",
  "gene": "UniProtKB:Q8IXA5",
  "term_id": "GO:0036126"
}